organellar chromatophore membrane [GO:0070112] (cellular component) Subtypes: organellar chromatophore inner membrane [GO:0070113], organellar chromatophore outer membrane [GO:0070114], organellar chromatophore thylakoid membrane [GO:0070118] Sources: GOC:mah Relationships: is_a cytoplasmic vesicle membrane [GO:0030659]; is part of organellar chromatophore [GO:0070111] Also known as: Paulinella-type chromatophore membrane Definition: Either of the lipid bilayers that surround an organellar chromatophore.